{
  "term_label": "DNA-binding transcription factor activity, RNA polymerase II-specific",
  "term_id": "GO:0000981",
  "gene_symbol": "GLIS2",
  "gene_name": "Zinc finger protein GLIS2",
  "gene": "UniProtKB:Q9BZE0"
}